{
  "gene_symbol": "CCDC82",
  "gene": "UniProtKB:Q8N4S0",
  "term_label": "nucleus",
  "gene_name": "Coiled-coil domain-containing protein 82",
  "term_id": "GO:0005634"
}